{
  "gene_symbol": "AK3",
  "term_label": "AMP metabolic process",
  "gene": "UniProtKB:Q9UIJ7",
  "term_id": "GO:0046033",
  "gene_name": "GTP:AMP phosphotransferase AK3, mitochondrial"
}